regulation of glial cell migration [GO:1903975] (biological process) Definition: Any process that modulates the frequency, rate or extent of glial cell migration. References: PMID:19100238 Sources: GOC:BHF, GOC:TermGenie, GOC:nc, GO_REF:0000058 Also known as: regulation of glia cell migration Relationships: is_a regulation of cell migration [GO:0030334]; regulates glial cell migration [GO:0008347] Subtypes: regulation of Schwann cell migration [GO:1900147], negative regulation of glial cell migration [GO:1903976], positive regulation of glial cell migration [GO:1903977], regulation of microglial cell migration [GO:1904139], GO:2000458